{
  "term_label": "nucleus",
  "gene_name": "Cysteine and glycine-rich protein 1",
  "gene_symbol": "CSRP1",
  "term_id": "GO:0005634",
  "gene": "UniProtKB:P21291"
}